{
  "gene_name": "Semaphorin-6B",
  "gene": "UniProtKB:Q9H3T3",
  "term_label": "axon guidance",
  "term_id": "GO:0007411",
  "gene_symbol": "SEMA6B"
}